{
  "gene_symbol": "SPON2",
  "gene_name": "Spondin-2",
  "gene": "UniProtKB:Q9BUD6",
  "term_id": "GO:0007155",
  "term_label": "cell adhesion"
}